{
  "gene": "UniProtKB:Q9Y4F4",
  "gene_name": "TOG array regulator of axonemal microtubules protein 1",
  "gene_symbol": "TOGARAM1",
  "term_label": "cilium",
  "term_id": "GO:0005929"
}